{
  "gene_name": "Keratin, type I cuticular Ha5",
  "term_label": "cytoskeleton",
  "gene": "UniProtKB:Q92764",
  "gene_symbol": "KRT35",
  "term_id": "GO:0005856"
}